{
  "term_label": "low-density lipoprotein particle clearance",
  "gene_name": "Platelet glycoprotein 4",
  "gene_symbol": "CD36",
  "gene": "UniProtKB:P16671",
  "term_id": "GO:0034383"
}